{
  "gene_symbol": "VPREB3",
  "gene": "UniProtKB:Q9UKI3",
  "term_label": "immunoglobulin complex",
  "term_id": "GO:0019814",
  "gene_name": "Pre-B lymphocyte protein 3"
}